{
  "gene": "UniProtKB:Q96A54",
  "gene_name": "Adiponectin receptor protein 1",
  "term_id": "GO:0005886",
  "term_label": "plasma membrane",
  "gene_symbol": "ADIPOR1"
}